{
  "gene_symbol": "CAV1",
  "term_id": "GO:0005901",
  "gene_name": "Caveolin-1",
  "gene": "UniProtKB:Q03135",
  "term_label": "caveola"
}